{
  "gene_name": "E3 SUMO-protein ligase RanBP2",
  "gene_symbol": "RANBP2",
  "term_label": "SUMO transferase activity",
  "term_id": "GO:0019789",
  "gene": "UniProtKB:P49792"
}